{
  "term_label": "positive regulation of cold-induced thermogenesis",
  "gene_name": "Transient receptor potential cation channel subfamily M member 8",
  "gene": "UniProtKB:Q7Z2W7",
  "term_id": "GO:0120162",
  "gene_symbol": "TRPM8"
}